{
  "gene": "UniProtKB:A6ND01",
  "gene_name": "Sperm-egg fusion protein Juno",
  "term_label": "sperm-egg recognition",
  "gene_symbol": "IZUMO1R",
  "term_id": "GO:0035036"
}